{
  "term_id": "GO:0000978",
  "gene_name": "Divergent paired-related homeobox",
  "gene_symbol": "DPRX",
  "term_label": "RNA polymerase II cis-regulatory region sequence-specific DNA binding",
  "gene": "UniProtKB:A6NFQ7"
}